{
  "gene_name": "Plectin",
  "gene_symbol": "PLEC",
  "term_id": "GO:0042060",
  "gene": "UniProtKB:Q15149",
  "term_label": "wound healing"
}